regulation of mitotic spindle elongation (spindle phase three) [GO:0110162] (biological process) References: PMID:27697865 Sources: GOC:vw Subtypes: negative regulation of mitotic spindle elongation (spindle phase three) [GO:0110163], positive regulation of mitotic spindle elongation (spindle phase three) [GO:0110164] Definition: Any process that modulates the frequency, rate or extent of the cell cycle process in which the distance is lengthened between poles of the mitotic spindle during mitotic anaphase B (spindle phase three). Relationships: is a type of GO:0032888; is_a regulation of mitotic spindle organization [GO:0060236]; regulates mitotic spindle elongation (spindle phase three) [GO:0061805]